negative regulation of satellite cell differentiation [GO:1902725] (BP) Also known as: down regulation of satellite cell differentiation, down-regulation of satellite cell differentiation, downregulation of satellite cell differentiation, inhibition of satellite cell differentiation References: PMID:23212449 Sources: GOC:TermGenie, GO_REF:0000058 Relationships: is a type of negative regulation of skeletal muscle cell differentiation [GO:2001015]; negatively regulates skeletal muscle satellite cell differentiation [GO:0014816] Definition: Any process that stops, prevents or reduces the frequency, rate or extent of satellite cell differentiation.